{
  "gene": "UniProtKB:Q86UV5",
  "term_label": "regulation of protein stability",
  "gene_name": "Ubiquitin carboxyl-terminal hydrolase 48",
  "term_id": "GO:0031647",
  "gene_symbol": "USP48"
}